{
  "gene_symbol": "CTNS",
  "gene_name": "Cystinosin",
  "term_label": "L-cystine transmembrane transporter activity",
  "term_id": "GO:0015184",
  "gene": "UniProtKB:O60931"
}